intracellular signal transduction [GO:0035556] (biological process) Sources: GOC:bf, GOC:jl, GOC:signaling, ISBN:3527303782 Subtypes: cell cycle checkpoint signaling [GO:0000075], phosphorelay signal transduction system [GO:0000160], ER-nucleus signaling pathway [GO:0006984], osmosensory signaling pathway [GO:0007231], chloroplast-nucleus signaling pathway [GO:0010019], intracellular receptor signaling pathway [GO:0030522], endoplasmic reticulum unfolded protein response [GO:0030968], stress-activated protein kinase signaling cascade [GO:0031098], GO:0031929, mitochondria-nucleus signaling pathway [GO:0031930], hippo signaling [GO:0035329], signal transduction in response to DNA damage [GO:0042770], phosphatidylinositol-mediated signaling [GO:0048015], RAM/MOR signaling [GO:0062200], protein kinase C signaling [GO:0070528], signal transduction by p53 class mediator [GO:0072331], intrinsic apoptotic signaling pathway [GO:0097193], GO:0097411, intracellular signaling cassette [GO:0141124] Also known as: intracellular signal transduction pathway, signal transmission via intracellular cascade, intracellular signaling cascade, intracellular signaling pathway Definition: The process in which a signal is passed on to downstream components within the cell, which become activated themselves to further propagate the signal and finally trigger a change in the function or state of the cell. Regulation: regulated by regulation of intracellular signal transduction [GO:1902531]; negatively regulated by negative regulation of intracellular signal transduction [GO:1902532]; positively regulated by positive regulation of intracellular signal transduction [GO:1902533] Relationships: is a type of signal transduction [GO:0007165]; occurs in intracellular anatomical structure [GO:0005622]